regulation of protein maturation [GO:1903317] (BP) Definition: Any process that modulates the frequency, rate or extent of protein maturation. Subtypes: GO:0070613, negative regulation of protein maturation [GO:1903318], positive regulation of protein maturation [GO:1903319], regulation of N-terminal peptidyl-methionine acetylation [GO:1904663], regulation of protein activation cascade [GO:2000257], regulation of N-terminal peptidyl-lysine acetylation [GO:2000759] Relationships: is a type of regulation of gene expression [GO:0010468]; is a type of regulation of protein metabolic process [GO:0051246]; regulates protein maturation [GO:0051604] Sources: GOC:TermGenie, GOC:vw, GO_REF:0000058